{
  "gene_symbol": "UFM1",
  "term_label": "Unknown molecular function",
  "gene": "UniProtKB:P61960",
  "term_id": "UNKNOWN:0001",
  "gene_name": "Ubiquitin-fold modifier 1"
}